{
  "gene_symbol": "TUBG2",
  "term_label": "mitotic cell cycle",
  "gene_name": "Tubulin gamma-2 chain",
  "term_id": "GO:0000278",
  "gene": "UniProtKB:Q9NRH3"
}